negative regulation of amine metabolic process [GO:0033239] (biological process) Sources: GOC:mah Definition: Any process that stops, prevents, or reduces the frequency, rate or extent of the chemical reactions and pathways involving amines. Subtypes: negative regulation of amine catabolic process [GO:0033242], negative regulation of dopamine metabolic process [GO:0045963], negative regulation of polyamine biosynthetic process [GO:0170066], GO:1900319, negative regulation of methane biosynthetic process from trimethylamine [GO:1900331], negative regulation of methane biosynthetic process from methylamine [GO:1900349] Also known as: negative regulation of amine metabolism, negative regulation of cellular amine metabolic process Relationships: is a type of negative regulation of metabolic process [GO:0009892]; is a type of regulation of amine metabolic process [GO:0033238]; negatively regulates amine metabolic process [GO:0009308]